{
  "term_id": "GO:0000398",
  "gene_name": "RNA-binding motif protein, X-linked 2",
  "term_label": "mRNA splicing, via spliceosome",
  "gene_symbol": "RBMX2",
  "gene": "UniProtKB:Q9Y388"
}